{
  "term_id": "GO:0005634",
  "gene_symbol": "ZNF329",
  "gene_name": "Zinc finger protein 329",
  "gene": "UniProtKB:Q86UD4",
  "term_label": "nucleus"
}